{
  "term_label": "Unknown molecular function",
  "term_id": "UNKNOWN:0001",
  "gene": "UniProtKB:P02749",
  "gene_name": "Beta-2-glycoprotein 1",
  "gene_symbol": "APOH"
}